{
  "term_label": "lysosome",
  "gene_name": "FYVE and coiled-coil domain-containing protein 1",
  "gene": "UniProtKB:Q9BQS8",
  "gene_symbol": "FYCO1",
  "term_id": "GO:0005764"
}